{
  "term_label": "GTPase activity",
  "gene_name": "Arf-GAP with GTPase, ANK repeat and PH domain-containing protein 4",
  "gene_symbol": "AGAP4",
  "term_id": "GO:0003924",
  "gene": "UniProtKB:Q96P64"
}